{
  "gene_symbol": "IGKV3-20",
  "gene_name": "Immunoglobulin kappa variable 3-20",
  "term_id": "GO:0019814",
  "term_label": "immunoglobulin complex",
  "gene": "UniProtKB:P01619"
}